regulation of cell septum assembly [GO:1901891] (biological process) Subtypes: GO:0032955, negative regulation of cell septum assembly [GO:1901892], positive regulation of cell septum assembly [GO:1901893] Definition: Any process that modulates the frequency, rate or extent of cell septum assembly. Relationships: is a type of regulation of cytokinetic process [GO:0032954]; is a type of regulation of cellular component biogenesis [GO:0044087]; is a type of regulation of cellular component organization [GO:0051128]; regulates cell septum assembly [GO:0090529] Sources: GOC:TermGenie